{
  "gene": "UniProtKB:Q1X8D7",
  "term_label": "Unknown molecular function",
  "gene_symbol": "LRRC36",
  "gene_name": "Leucine-rich repeat-containing protein 36",
  "term_id": "UNKNOWN:0001"
}